extracellular membrane-bounded organelle [GO:0065010] (CC) Subtypes: extracellular vesicle [GO:1903561] Sources: GOC:isa_complete Definition: Organized structure of distinctive morphology and function, bounded by a lipid bilayer membrane and occurring outside the cell. Also known as: extracellular membrane-enclosed organelle Relationships: is a type of membrane-bounded organelle [GO:0043227]; is a type of GO:0043230